{
  "term_label": "calcium ion transmembrane transport",
  "gene_symbol": "P2RX5",
  "term_id": "GO:0070588",
  "gene_name": "P2X purinoceptor 5",
  "gene": "UniProtKB:Q93086"
}